{
  "gene_symbol": "NEFH",
  "gene": "UniProtKB:P12036",
  "gene_name": "Neurofilament heavy polypeptide",
  "term_label": "intermediate filament bundle assembly",
  "term_id": "GO:0045110"
}